{
  "gene_symbol": "TADA3",
  "term_label": "SAGA complex",
  "gene_name": "Transcriptional adapter 3",
  "term_id": "GO:0000124",
  "gene": "UniProtKB:O75528"
}